extrinsic component of mitochondrial outer membrane [GO:0031315] (cellular component) Also known as: extrinsic to mitochondrial outer membrane Sources: GOC:dos, GOC:mah Relationships: is a type of extrinsic component of organelle membrane [GO:0031312]; BFO_0000050 mitochondrial outer membrane [GO:0005741] Definition: The component of a mitochondrial outer membrane consisting of gene products and protein complexes that are loosely bound to one of its surfaces, but not integrated into the hydrophobic region.